dendritic spine cytoplasm [GO:0061846] (cellular component) Relationships: is a type of dendrite cytoplasm [GO:0032839]; is part of GO:0043197 Definition: The region of the neuronal cytoplasm located in dendritic spines. References: PMID:15673667